{
  "term_label": "Unknown molecular function",
  "term_id": "UNKNOWN:0001",
  "gene_symbol": "MRPL30",
  "gene_name": "Large ribosomal subunit protein uL30m",
  "gene": "UniProtKB:Q8TCC3"
}